{
  "gene": "UniProtKB:P49770",
  "term_label": "eukaryotic translation initiation factor 2B complex",
  "term_id": "GO:0005851",
  "gene_symbol": "EIF2B2",
  "gene_name": "Translation initiation factor eIF-2B subunit beta"
}